tRNA 2'-O-methyltransferase activity [GO:0106050] (MF) Definition: Catalysis of the reaction: S-adenosyl-L-methionine + tRNA = S-adenosyl-L-homocysteine + tRNA containing a 2'-O-nucleotide. Relationships: is a type of tRNA methyltransferase activity [GO:0008175]; is a type of RNA 2'-O-methyltransferase activity [GO:0062105] References: PMID:17242307